{
  "gene_name": "Dickkopf-related protein 4",
  "term_label": "extracellular space",
  "gene": "UniProtKB:Q9UBT3",
  "gene_symbol": "DKK4",
  "term_id": "GO:0005615"
}